beta-L-arabinosidase activity [GO:0047701] (molecular function) Also known as: b-L-arabinosidase activity, beta-L-arabinoside arabinohydrolase activity, vicianosidase activity Relationships: is a type of hydrolase activity, hydrolyzing O-glycosyl compounds [GO:0004553] Sources: EC:3.2.1.88 Definition: Catalysis of the reaction: H2O + a beta-L-arabinoside = L-arabinose + an alcohol.